ciliary tip [GO:0097542] (cellular component) Definition: Part of the cilium where the axoneme ends. The ciliary tip has been implicated in ciliary assembly and disassembly, as well as signal transduction. Relationships: is a type of cellular anatomical structure [GO:0110165]; is part of cilium [GO:0005929] Note: Note that cilia and eukaryotic flagella are deemed to be equivalent. Also known as: cilial tip, cilium tip, flagellar tip, flagellum tip References: PMID:23970417 Sources: GOC:cilia